{
  "gene": "UniProtKB:A0A075B6N4",
  "gene_name": "T cell receptor beta variable 25-1",
  "term_id": "GO:0007166",
  "gene_symbol": "TRBV25-1",
  "term_label": "cell surface receptor signaling pathway"
}